{
  "gene_symbol": "CNEP1R1",
  "gene": "UniProtKB:Q8N9A8",
  "gene_name": "Nuclear envelope phosphatase-regulatory subunit 1",
  "term_label": "cytoplasm",
  "term_id": "GO:0005737"
}